{
  "term_id": "GO:0042073",
  "gene_symbol": "TRAF3IP1",
  "term_label": "intraciliary transport",
  "gene": "UniProtKB:Q8TDR0",
  "gene_name": "TRAF3-interacting protein 1"
}